{
  "term_label": "Unknown cellular component",
  "gene": "UniProtKB:Q9NTX9",
  "gene_name": "Protein FAM217B",
  "gene_symbol": "FAM217B",
  "term_id": "UNKNOWN:0003"
}